guanyl ribonucleotide binding [GO:0032561] (molecular function) Sources: GOC:mah Subtypes: GTP binding [GO:0005525], GMP binding [GO:0019002], GDP binding [GO:0019003], cGMP binding [GO:0030553], cyclic-di-GMP binding [GO:0035438], GO:0061507, guanosine tetraphosphate binding [GO:0097216], 3',3'-cyclic GMP-AMP binding [GO:0140703] Definition: Binding to a guanyl ribonucleotide, any compound consisting of guanosine esterified with (ortho)phosphate or an oligophosphate at any hydroxyl group on the ribose moiety. Relationships: is a type of guanyl nucleotide binding [GO:0019001]; is_a purine ribonucleotide binding [GO:0032555]